{
  "term_label": "plasma membrane",
  "gene_symbol": "RAB5C",
  "gene": "UniProtKB:P51148",
  "term_id": "GO:0005886",
  "gene_name": "Ras-related protein Rab-5C"
}